{
  "gene_name": "Vascular endothelial growth factor receptor 1",
  "gene_symbol": "FLT1",
  "gene": "UniProtKB:P17948",
  "term_label": "positive regulation of cell migration",
  "term_id": "GO:0030335"
}